recycling endosome [GO:0055037] (cellular component) Definition: An organelle consisting of a network of tubules that functions in targeting molecules, such as receptors transporters and lipids, to the plasma membrane. References: PMID:10930469, PMID:15601896, PMID:16246101, PMID:21556374, PMID:21562044 Sources: GOC:dph, GOC:jid, GOC:kmv, GOC:rph Also known as: endosomal recycling compartment, ERC, endosome recycling compartment Relationships: is a type of endosome [GO:0005768] Subtypes: apical recycling endosome [GO:0090653], basolateral recycling endosome [GO:0090654], peri-centrosomal recycling endosome [GO:0098832], GO:0098837